{
  "gene_symbol": "TRAJ50",
  "term_label": "Unknown molecular function",
  "gene_name": "T cell receptor alpha joining 50 (Fragment)",
  "term_id": "UNKNOWN:0001",
  "gene": "UniProtKB:A0A075B6X7"
}